nuclear outer membrane-endoplasmic reticulum membrane network [GO:0042175] (cellular component) Definition: The continuous network of membranes encompassing the nuclear outer membrane and the endoplasmic reticulum membrane. Sources: GOC:bf, GOC:jl, GOC:mah, GOC:mcc, GOC:pr Also known as: nuclear membrane-ER network, nuclear membrane-endoplasmic reticulum continuum, NE-ER continuum, NE-ER network, nuclear envelope-ER network, nuclear envelope-endoplasmic reticulum continuum, nuclear envelope-endoplasmic reticulum network Relationships: is_a membrane [GO:0016020]; is part of GO:0012505